{
  "term_label": "DNA-binding transcription factor activity, RNA polymerase II-specific",
  "gene": "UniProtKB:Q9Y2Y9",
  "gene_name": "Krueppel-like factor 13",
  "gene_symbol": "KLF13",
  "term_id": "GO:0000981"
}